liver morphogenesis [GO:0072576] (biological process) Relationships: is a type of gland morphogenesis [GO:0022612]; is part of GO:0001889 Sources: GOC:mah Definition: The process in which the anatomical structures of the liver are generated and organized.